{
  "gene_symbol": "KIF20B",
  "term_label": "kinesin complex",
  "gene_name": "Kinesin-like protein KIF20B",
  "term_id": "GO:0005871",
  "gene": "UniProtKB:Q96Q89"
}